{
  "gene_symbol": "H3C13",
  "term_label": "structural constituent of chromatin",
  "gene": "UniProtKB:Q71DI3",
  "term_id": "GO:0030527",
  "gene_name": "Histone H3.2"
}